{
  "term_label": "Unknown molecular function",
  "gene": "UniProtKB:Q9BRT2",
  "gene_symbol": "UQCC2",
  "term_id": "UNKNOWN:0001",
  "gene_name": "Ubiquinol-cytochrome-c reductase complex assembly factor 2"
}